{
  "term_label": "Unknown cellular component",
  "gene_name": "Submaxillary gland androgen-regulated protein 3B",
  "term_id": "UNKNOWN:0003",
  "gene_symbol": "SMR3B",
  "gene": "UniProtKB:P02814"
}